{
  "gene": "UniProtKB:Q8IZ08",
  "gene_symbol": "GPR135",
  "term_label": "G protein-coupled receptor signaling pathway",
  "gene_name": "G-protein coupled receptor 135",
  "term_id": "GO:0007186"
}